{
  "term_label": "endoplasmic reticulum",
  "gene_symbol": "METTL9",
  "term_id": "GO:0005783",
  "gene": "UniProtKB:Q9H1A3",
  "gene_name": "Protein-L-histidine N-pros-methyltransferase"
}